arogenate dehydrogenase (NADP+) activity [GO:0033730] (molecular function) Definition: Catalysis of the reaction: L-arogenate + NADP+ = L-tyrosine + NADPH + CO2. Relationships: is a type of arogenate dehydrogenase [NAD(P)+] activity [GO:0033731] Also known as: arogenic dehydrogenase activity, pretyrosine dehydrogenase activity, L-arogenate:NADP+ oxidoreductase (decarboxylating) activity, TyrAAT1, TyrAAT2, TyrAa Sources: EC:1.3.1.78